{
  "gene_name": "Phosphomannomutase 2",
  "gene": "UniProtKB:O15305",
  "term_id": "GO:0004615",
  "term_label": "phosphomannomutase activity",
  "gene_symbol": "PMM2"
}